{
  "gene_name": "Small cysteine and glycine repeat-containing protein 3",
  "gene": "UniProtKB:A0A286YF60",
  "term_label": "Unknown biological process",
  "gene_symbol": "SCYGR3",
  "term_id": "UNKNOWN:0002"
}